{
  "gene_symbol": "SPAG9",
  "gene": "UniProtKB:O60271",
  "term_label": "vesicle-mediated transport",
  "gene_name": "C-Jun-amino-terminal kinase-interacting protein 4",
  "term_id": "GO:0016192"
}